regulation of nuclear migration along microtubule [GO:1902838] (biological process) Subtypes: negative regulation of nuclear migration along microtubule [GO:1902839], positive regulation of nuclear migration along microtubule [GO:1902840], regulation of nuclear migration during mitotic telophase [GO:1902852] Definition: Any process that modulates the frequency, rate or extent of nuclear migration along microtubule. References: PMID:23087209 Sources: GOC:TermGenie, GO_REF:0000058 Also known as: regulation of nuclear movement, microtubule-mediated, regulation of nucleus migration, regulation of microtubule cytoskeleton-dependent nuclear positioning, regulation of microtubule cytoskeleton-dependent nucleus positioning, regulation of microtubule-dependent nuclear positioning, regulation of microtubule-dependent nucleus positioning, regulation of microtubule-mediated nuclear migration, regulation of nuclear migration, microtubule-mediated, regulation of transport of nucleus by microtubules, regulation of transport of nucleus, microtubule-mediated Relationships: is a type of regulation of organelle transport along microtubule [GO:1902513]; regulates nuclear migration along microtubule [GO:0030473]